{
  "gene_name": "Aromatase",
  "term_id": "GO:0005783",
  "gene_symbol": "CYP19A1",
  "gene": "UniProtKB:P11511",
  "term_label": "endoplasmic reticulum"
}